oxidoreductase activity, acting on a sulfur group of donors, iron-sulfur protein as acceptor [GO:0016673] (molecular function) Also known as: oxidoreductase activity, acting on sulphur group of donors, iron-sulphur protein as acceptor Relationships: is a type of GO:0016667 Sources: GOC:jl Definition: Catalysis of an oxidation-reduction (redox) reaction in which a sulfur-containing group acts as a hydrogen or electron donor and reduces an iron-sulfur protein. Subtypes: GO:0050311, ferredoxin-thioredoxin reductase activity [GO:0103012]